{
  "gene_symbol": "PPP2R5E",
  "term_id": "UNKNOWN:0002",
  "gene_name": "Serine_threonine-protein phosphatase 2A 56 kDa regulatory subunit epsilon isoform",
  "term_label": "Unknown biological process",
  "gene": "UniProtKB:Q16537"
}